{
  "gene_name": "Defensin alpha 4",
  "term_label": "antibacterial humoral response",
  "term_id": "GO:0019731",
  "gene_symbol": "DEFA4",
  "gene": "UniProtKB:P12838"
}